regulation of neurogenesis [GO:0050767] (BP) Sources: GOC:ai Subtypes: regulation of gliogenesis [GO:0014013], negative regulation of neurogenesis [GO:0050768], positive regulation of neurogenesis [GO:0050769] Definition: Any process that modulates the frequency, rate or extent of neurogenesis, the generation of cells in the nervous system. Relationships: is a type of GO:0051960; is a type of GO:0060284; regulates neurogenesis [GO:0022008]